{
  "term_id": "GO:0000978",
  "gene_name": "Zinc finger protein 23",
  "gene_symbol": "ZNF23",
  "gene": "UniProtKB:P17027",
  "term_label": "RNA polymerase II cis-regulatory region sequence-specific DNA binding"
}